{
  "gene": "UniProtKB:Q9Y6K5",
  "term_id": "GO:0005654",
  "gene_symbol": "OAS3",
  "gene_name": "2'-5'-oligoadenylate synthase 3",
  "term_label": "nucleoplasm"
}